purine deoxyribonucleoside monophosphate metabolic process [GO:0009170] (biological process) Definition: The chemical reactions and pathways involving purine deoxyribonucleoside monophosphate, a compound consisting of a purine base linked to a deoxyribose sugar esterified with phosphate on the sugar. Also known as: purine deoxyribonucleoside monophosphate metabolism Subtypes: purine deoxyribonucleoside monophosphate biosynthetic process [GO:0009171], purine deoxyribonucleoside monophosphate catabolic process [GO:0009172], GO:0046053, GO:0046054 Sources: GOC:go_curators, ISBN:0198506732 Relationships: is a type of purine nucleoside monophosphate metabolic process [GO:0009126]